{
  "term_label": "Unknown molecular function",
  "term_id": "UNKNOWN:0001",
  "gene_name": "Integrator complex subunit 4",
  "gene_symbol": "INTS4",
  "gene": "UniProtKB:Q96HW7"
}